{
  "term_id": "GO:0000122",
  "gene_symbol": "LIN37",
  "gene": "UniProtKB:Q96GY3",
  "gene_name": "Protein lin-37 homolog",
  "term_label": "negative regulation of transcription by RNA polymerase II"
}